{
  "term_id": "UNKNOWN:0002",
  "term_label": "Unknown biological process",
  "gene": "UniProtKB:Q8N9R6",
  "gene_symbol": "CDRT4",
  "gene_name": "CMT1A duplicated region transcript 4 protein"
}